{
  "gene": "UniProtKB:P10072",
  "term_id": "GO:0000981",
  "gene_symbol": "ZNF875",
  "gene_name": "Zinc finger protein 875",
  "term_label": "DNA-binding transcription factor activity, RNA polymerase II-specific"
}